{
  "gene_symbol": "TAS2R1",
  "term_id": "GO:0033038",
  "gene_name": "Taste receptor type 2 member 1",
  "gene": "UniProtKB:Q9NYW7",
  "term_label": "bitter taste receptor activity"
}